{
  "gene": "UniProtKB:Q96EY5",
  "gene_symbol": "MVB12A",
  "term_id": "GO:0032510",
  "gene_name": "Multivesicular body subunit 12A",
  "term_label": "endosome to lysosome transport via multivesicular body sorting pathway"
}